{
  "gene_name": "Solute carrier family 23 member 2",
  "term_label": "apical plasma membrane",
  "gene_symbol": "SLC23A2",
  "term_id": "GO:0016324",
  "gene": "UniProtKB:Q9UGH3"
}